{
  "term_id": "GO:0005783",
  "gene_name": "Protein O-linked-mannose beta-1,4-N-acetylglucosaminyltransferase 2",
  "gene_symbol": "POMGNT2",
  "term_label": "endoplasmic reticulum",
  "gene": "UniProtKB:Q8NAT1"
}